{
  "gene_name": "Histone H2B type 1-O",
  "term_label": "antimicrobial humoral immune response mediated by antimicrobial peptide",
  "gene_symbol": "H2BC17",
  "term_id": "GO:0061844",
  "gene": "UniProtKB:P23527"
}